{
  "gene_name": "Polypeptide N-acetylgalactosaminyltransferase 6",
  "term_label": "protein O-linked glycosylation",
  "gene_symbol": "GALNT6",
  "gene": "UniProtKB:Q8NCL4",
  "term_id": "GO:0006493"
}